{
  "term_label": "Unknown cellular component",
  "term_id": "UNKNOWN:0003",
  "gene_name": "Forkhead box protein D4-like 1",
  "gene": "UniProtKB:Q9NU39",
  "gene_symbol": "FOXD4L1"
}